{
  "term_id": "GO:0051604",
  "gene_name": "Tetraspanin-33",
  "term_label": "protein maturation",
  "gene": "UniProtKB:Q86UF1",
  "gene_symbol": "TSPAN33"
}